D-series resolvin biosynthetic process [GO:0106296] (biological process) Relationships: is a type of resolvin biosynthetic process [GO:0106295] References: PMID:12391014 Definition: The chemical reactions and pathways resulting in the formation of resolvin family D-series, hydroxy fatty acids derived from docosahexaenoic acid.